iron-sulfur cluster chaperone activity [GO:0140132] (molecular function) References: PMID:22966982, PMID:29051382 Also known as: iron-sulfur cluster carrier activity Relationships: is a type of metallochaperone activity [GO:0016530]; has part iron-sulfur cluster binding [GO:0051536] Definition: Binding to an iron-sulfur cluster and delivering it to an acceptor molecule.